{
  "term_label": "nuclear pore central transport channel",
  "gene": "UniProtKB:P37198",
  "term_id": "GO:0044613",
  "gene_symbol": "NUP62",
  "gene_name": "Nuclear pore glycoprotein p62"
}